{
  "gene_name": "Putative uncharacterized protein encoded by LINC00312",
  "gene": "UniProtKB:Q9Y6C7",
  "gene_symbol": "LINC00312",
  "term_id": "UNKNOWN:0001",
  "term_label": "Unknown molecular function"
}